{
  "term_id": "UNKNOWN:0001",
  "gene_symbol": "CT45A3",
  "gene": "UniProtKB:Q8NHU0",
  "term_label": "Unknown molecular function",
  "gene_name": "Cancer_testis antigen family 45 member A3"
}